{
  "gene_name": "Tyrosine-protein phosphatase non-receptor type 22",
  "term_id": "GO:0045088",
  "gene_symbol": "PTPN22",
  "term_label": "regulation of innate immune response",
  "gene": "UniProtKB:Q9Y2R2"
}